dehydro-L-gulonate decarboxylase activity [GO:0047842] (molecular function) Sources: EC:4.1.1.34, RHEA:11084 Relationships: is a type of carboxy-lyase activity [GO:0016831] Definition: Catalysis of the reaction: 3-dehydro-L-gulonate + H+ = L-xylulose + CO2. Also known as: 3-dehydro-L-gulonate carboxy-lyase (L-xylulose-forming), 3-dehydro-L-gulonate carboxy-lyase activity, 3-keto-L-gulonate decarboxylase activity, keto-L-gulonate decarboxylase activity